{
  "gene_symbol": "LDLRAD4",
  "term_id": "GO:0031901",
  "gene": "UniProtKB:O15165",
  "term_label": "early endosome membrane",
  "gene_name": "Low-density lipoprotein receptor class A domain-containing protein 4"
}